transitional one stage B cell differentiation [GO:0002333] (biological process) Note: Note that immunologists typically use the word 'development' to refer to cells of B or T cell lineages undergoing the process that GO describes as 'cell differentiation'. Relationships: is a type of transitional stage B cell differentiation [GO:0002332] Definition: The process in which immature B cells from the bone marrow acquire the specialized features of T1 stage B cells in the spleen. T1 stage B cells do not express either CD23 or CD21. Sources: GOC:jal, ISBN:0781735149 Also known as: T1 stage B cell differentiation, transitional one stage B lymphocyte differentiation, transitional one stage B-cell differentiation, transitional one stage B-lymphocyte differentiation, transitional one stage B cell development